{
  "gene": "UniProtKB:Q8N2I9",
  "term_id": "GO:0043408",
  "term_label": "regulation of MAPK cascade",
  "gene_name": "Serine_threonine-protein kinase 40",
  "gene_symbol": "STK40"
}